box H/ACA telomerase RNP complex [GO:0090661] (cellular component) References: PMID:22527283 Sources: GOC:BHF, GOC:BHF_telomere, GOC:jbu Relationships: is a type of box H/ACA RNP complex [GO:0072588]; is a type of GO:0140513; BFO_0000050 GO:0005697 Definition: A box H/ACA ribonucleoprotein complex that contains the RNA component of vertebrate telomerase, the enzyme essential for the replication of chromosome termini in most eukaryotes. This ribonucleoprotein complex is a structural box H/ACA RNP, which does not have the catalytic pseudouridylation function shared by the majority of H/ACA RNPs present in the cell.